{
  "gene_name": "RNA polymerase II subunit A C-terminal domain phosphatase SSU72 like protein 1",
  "term_id": "GO:0006369",
  "term_label": "termination of RNA polymerase II transcription",
  "gene": "UniProtKB:A0A1W2PQ27",
  "gene_symbol": "SSU72L1"
}